{
  "gene_symbol": "CKAP2L",
  "gene_name": "Cytoskeleton-associated protein 2-like",
  "term_id": "UNKNOWN:0001",
  "term_label": "Unknown molecular function",
  "gene": "UniProtKB:Q8IYA6"
}